{
  "term_id": "GO:0005902",
  "gene_symbol": "MYO7A",
  "term_label": "microvillus",
  "gene_name": "Unconventional myosin-VIIa",
  "gene": "UniProtKB:Q13402"
}